{
  "gene_name": "Left-right determination factor 1",
  "term_id": "GO:0005615",
  "term_label": "extracellular space",
  "gene": "UniProtKB:O75610",
  "gene_symbol": "LEFTY1"
}